{
  "gene_symbol": "PTAFR",
  "gene": "UniProtKB:P25105",
  "gene_name": "Platelet-activating factor receptor",
  "term_id": "GO:0007186",
  "term_label": "G protein-coupled receptor signaling pathway"
}